{
  "gene_symbol": "OR2A25",
  "gene_name": "Olfactory receptor",
  "term_id": "UNKNOWN:0001",
  "gene": "UniProtKB:A0A126GWI2",
  "term_label": "Unknown molecular function"
}